GDP-mannose transmembrane transporter activity [GO:0005458] (molecular function) Definition: Enables the transfer of a GDP-mannose from one side of a membrane to the other. GDP-mannose is a substance composed of mannose in glycosidic linkage with guanosine diphosphate. Sources: GOC:ai, GOC:mtg_transport, ISBN:0815340729 Relationships: is_a GO:0036080; is part of GO:1990570